{
  "gene_symbol": "UCP3",
  "term_id": "GO:0015078",
  "gene": "UniProtKB:P55916",
  "term_label": "proton transmembrane transporter activity",
  "gene_name": "Putative mitochondrial transporter UCP3"
}